{
  "gene": "UniProtKB:O15520",
  "gene_name": "Fibroblast growth factor 10",
  "term_label": "neurogenesis",
  "term_id": "GO:0022008",
  "gene_symbol": "FGF10"
}